{
  "gene_symbol": "ANKRD20A2P",
  "term_id": "UNKNOWN:0001",
  "gene": "UniProtKB:Q5SQ80",
  "gene_name": "Putative ankyrin repeat domain-containing protein 20A2",
  "term_label": "Unknown molecular function"
}